dermatan sulfate proteoglycan catabolic process [GO:0030209] (biological process) Definition: The chemical reactions and pathways resulting in the breakdown of dermatan sulfate proteoglycans, which consist of a core protein linked to a dermatan sulfate glycosaminoglycan. The dermatan sulfate chain is composed of the repeating disaccharide unit beta-(1,4)-D-hexuronic acid-beta-(1,3)-N-acetyl-D-galactosamine. The former can be a mixture of sulfated and nonsulfated D-glucuronic and L-iduronic acids and the latter can be O-sulfated. Relationships: is a type of proteoglycan catabolic process [GO:0030167]; is a type of dermatan sulfate proteoglycan metabolic process [GO:0050655] Also known as: chondroitin sulfate B catabolic process, chondroitin sulfate B catabolism, dermatan sulfate breakdown, dermatan sulfate catabolism, dermatan sulfate degradation, dermatan sulphate catabolic process, dermatan sulphate catabolism References: PMID:17239763